{
  "gene_symbol": "KANSL2",
  "gene": "UniProtKB:Q9H9L4",
  "term_label": "Unknown molecular function",
  "gene_name": "KAT8 regulatory NSL complex subunit 2",
  "term_id": "UNKNOWN:0001"
}